{
  "term_label": "spermatid nucleus differentiation",
  "term_id": "GO:0007289",
  "gene_name": "Arf-GAP domain and FG repeat-containing protein 2",
  "gene": "UniProtKB:O95081",
  "gene_symbol": "AGFG2"
}